{
  "term_id": "UNKNOWN:0002",
  "term_label": "Unknown biological process",
  "gene_name": "Proline-rich protein 22",
  "gene": "UniProtKB:Q8IZ63",
  "gene_symbol": "PRR22"
}